{
  "term_label": "inhibitory MHC class I receptor activity",
  "term_id": "GO:0032396",
  "gene": "UniProtKB:O75022",
  "gene_name": "Leukocyte immunoglobulin-like receptor subfamily B member 3",
  "gene_symbol": "LILRB3"
}